{
  "gene_symbol": "PNRC1",
  "gene_name": "Proline-rich nuclear receptor coactivator 1",
  "term_id": "GO:0005634",
  "gene": "UniProtKB:Q12796",
  "term_label": "nucleus"
}